positive regulation of inhibin secretion [GO:0032340] (biological process) Definition: Any process that activates or increases the frequency, rate or extent of the regulated release of inhibin from a cell. Sources: GOC:mah Also known as: up regulation of inhibin secretion, up-regulation of inhibin secretion, upregulation of inhibin secretion, activation of inhibin secretion, stimulation of inhibin secretion Relationships: is_a GO:0032338; is a type of positive regulation of hormone secretion [GO:0046887]; RO_0002213 inhibin secretion [GO:0032334]